{
  "gene_symbol": "SYNPO",
  "gene_name": "Synaptopodin",
  "term_id": "GO:0097444",
  "gene": "UniProtKB:Q8N3V7",
  "term_label": "spine apparatus"
}